{
  "gene_symbol": "LGALS7",
  "term_id": "GO:0030246",
  "term_label": "carbohydrate binding",
  "gene_name": "Galectin-7",
  "gene": "UniProtKB:P47929"
}